pathogen-containing vacuole [GO:0140220] (cellular component) References: PMID:10560000, PMID:26842840 Subtypes: GO:0039679 Also known as: pathogen inclusion, pathogen-containing compartment Relationships: is a type of host cell part [GO:0033643] Definition: A membrane-bound intracellular compartment that is formed upon internalization of a pathogen into a host cell, and in which the pathogen resides.